{
  "term_id": "GO:0031492",
  "gene_name": "Histone H1.3",
  "term_label": "nucleosomal DNA binding",
  "gene": "UniProtKB:P16402",
  "gene_symbol": "H1-3"
}